{
  "term_id": "GO:0000978",
  "gene_name": "Myoblast determination protein 1",
  "term_label": "RNA polymerase II cis-regulatory region sequence-specific DNA binding",
  "gene_symbol": "MYOD1",
  "gene": "UniProtKB:P15172"
}